{
  "gene_name": "N-arachidonyl glycine receptor",
  "gene_symbol": "GPR18",
  "gene": "UniProtKB:Q14330",
  "term_id": "GO:0004930",
  "term_label": "G protein-coupled receptor activity"
}